{
  "gene_symbol": "NUDC",
  "gene": "UniProtKB:Q9Y266",
  "gene_name": "Nuclear migration protein nudC",
  "term_label": "cytoplasm",
  "term_id": "GO:0005737"
}